{
  "term_id": "GO:0005685",
  "term_label": "U1 snRNP",
  "gene_name": "Small nuclear ribonucleoprotein E",
  "gene": "UniProtKB:P62304",
  "gene_symbol": "SNRPE"
}